{
  "gene_symbol": "NR1H2",
  "gene_name": "Oxysterols receptor LXR-beta",
  "gene": "UniProtKB:P55055",
  "term_id": "GO:0000978",
  "term_label": "RNA polymerase II cis-regulatory region sequence-specific DNA binding"
}